{
  "gene_name": "Cytochrome c oxidase assembly protein COX18, mitochondrial",
  "gene": "UniProtKB:Q8N8Q8",
  "gene_symbol": "COX18",
  "term_id": "GO:0005743",
  "term_label": "mitochondrial inner membrane"
}